{
  "gene": "UniProtKB:Q9Y385",
  "gene_symbol": "UBE2J1",
  "term_id": "GO:0061631",
  "gene_name": "Ubiquitin-conjugating enzyme E2 J1",
  "term_label": "ubiquitin conjugating enzyme activity"
}